positive regulation of transepithelial migration of symbiont in host [GO:0140471] (biological process) References: PMID:29113016 Definition: Any process that activates or increases the frequency, rate or extent of transepithelial migration of symbiont in host. Also known as: positive regulation of symbiont-mediated migration across host transepithelium, positive regulation of symbiont-mediated migration through host transepithelium, positive regulation of transmigration of symbiont in host Relationships: is a type of GO:0043903; is a type of positive regulation of biological process [GO:0048518]; positively regulates symbiont-mediated migration across host transepithelium [GO:0035756]